{
  "gene_symbol": "CILK1",
  "gene": "UniProtKB:Q9UPZ9",
  "term_label": "cilium assembly",
  "term_id": "GO:0060271",
  "gene_name": "Serine_threonine-protein kinase ICK"
}